{
  "term_label": "negative regulation of translational initiation",
  "gene": "UniProtKB:P0DMB2",
  "gene_name": "Uncharacterized protein C8orf88",
  "gene_symbol": "C8orf88",
  "term_id": "GO:0045947"
}